cell cycle G1/S phase transition [GO:0044843] (biological process) Sources: GOC:mtg_cell_cycle Definition: The cell cycle process by which a cell in G1 phase commits to S phase. Relationships: is a type of cell cycle phase transition [GO:0044770] Subtypes: G1/S transition of mitotic cell cycle [GO:0000082] Regulation: regulated by regulation of cell cycle G1/S phase transition [GO:1902806]; negatively regulated by negative regulation of cell cycle G1/S phase transition [GO:1902807]; positively regulated by positive regulation of cell cycle G1/S phase transition [GO:1902808]